{
  "term_id": "GO:0090694",
  "gene": "UniProtKB:Q6KC79",
  "gene_name": "Nipped-B-like protein",
  "gene_symbol": "NIPBL",
  "term_label": "Scc2-Scc4 cohesin loading complex"
}